{
  "term_id": "GO:0032040",
  "gene_name": "rRNA-processing protein UTP23 homolog",
  "term_label": "small-subunit processome",
  "gene": "UniProtKB:Q9BRU9",
  "gene_symbol": "UTP23"
}